{
  "gene": "UniProtKB:Q96QK1",
  "gene_name": "Vacuolar protein sorting-associated protein 35",
  "term_label": "retrograde transport, endosome to Golgi",
  "term_id": "GO:0042147",
  "gene_symbol": "VPS35"
}